{
  "gene": "UniProtKB:P05015",
  "gene_name": "Interferon alpha-16",
  "term_label": "T cell activation involved in immune response",
  "term_id": "GO:0002286",
  "gene_symbol": "IFNA16"
}